{
  "gene": "UniProtKB:P23141",
  "gene_symbol": "CES1",
  "term_label": "lipid droplet",
  "gene_name": "Liver carboxylesterase 1",
  "term_id": "GO:0005811"
}